red light photoreceptor activity [GO:0031517] (molecular function) Definition: The function of absorbing and responding to electromagnetic radiation with a wavelength of approximately 660nm. The response may involve a change in conformation. Sources: GOC:nln Relationships: is a type of red or far-red light photoreceptor activity [GO:0009883]; is part of red light signaling pathway [GO:0010161]